{
  "gene": "UniProtKB:O14512",
  "gene_symbol": "SOCS7",
  "term_label": "signaling adaptor activity",
  "gene_name": "Suppressor of cytokine signaling 7",
  "term_id": "GO:0035591"
}